bacterial biofilm matrix surface [GO:0097313] (cellular component) Relationships: is a type of GO:0110165; is part of GO:0097311 References: PMID:22571672 Sources: GOC:imk, Wikipedia:Biofilm Definition: The external part of the biofilm matrix, a structure lying external to bacterial cells. A biofilm is an aggregate of surface-associated bacteria, and the biofilm matrix is the envelope of polymeric substances that surrounds the bacteria.